regulation of emericellamide A biosynthetic process [GO:1900661] (biological process) Sources: GOC:TermGenie, GOC:di Also known as: regulation of emericellamide A anabolism, regulation of emericellamide A biosynthesis, regulation of emericellamide A formation, regulation of emericellamide A synthesis Subtypes: GO:1900662, GO:1900663 Relationships: is a type of regulation of emericellamide biosynthetic process [GO:1900658]; regulates emericellamide A biosynthetic process [GO:1900617] Definition: Any process that modulates the frequency, rate or extent of emericellamide A biosynthetic process.